regulation of mesenchymal stem cell differentiation [GO:2000739] (biological process) Subtypes: negative regulation of mesenchymal stem cell differentiation [GO:2000740], positive regulation of mesenchymal stem cell differentiation [GO:2000741], regulation of amniotic stem cell differentiation [GO:2000797] Sources: GOC:obol Relationships: is a type of regulation of stem cell differentiation [GO:2000736]; regulates mesenchymal stem cell differentiation [GO:0072497] Definition: Any process that modulates the frequency, rate or extent of mesenchymal stem cell differentiation.